{
  "term_label": "positive regulation of DNA-templated transcription",
  "gene_symbol": "NUP85",
  "gene_name": "Nuclear pore complex protein Nup85",
  "term_id": "GO:0045893",
  "gene": "UniProtKB:Q9BW27"
}